{
  "gene_symbol": "ARHGEF17",
  "term_label": "cytoplasm",
  "gene": "UniProtKB:Q96PE2",
  "gene_name": "Rho guanine nucleotide exchange factor 17",
  "term_id": "GO:0005737"
}